{
  "gene": "UniProtKB:P28074",
  "term_id": "GO:0019774",
  "term_label": "proteasome core complex, beta-subunit complex",
  "gene_symbol": "PSMB5",
  "gene_name": "Proteasome subunit beta type-5"
}